{
  "term_id": "GO:0006003",
  "gene_symbol": "PFKFB3",
  "gene": "UniProtKB:Q16875",
  "gene_name": "6-phosphofructo-2-kinase_fructose-2,6-bisphosphatase 3",
  "term_label": "fructose 2,6-bisphosphate metabolic process"
}